{
  "gene": "UniProtKB:Q6ZPD8",
  "gene_symbol": "DGAT2L6",
  "term_id": "GO:0008374",
  "term_label": "O-acyltransferase activity",
  "gene_name": "Diacylglycerol O-acyltransferase 2-like protein 6"
}